2-oxoglutarate synthase activity [GO:0047553] (molecular function) Sources: EC:1.2.7.3, MetaCyc:2-OXOGLUTARATE-SYNTHASE-RXN Relationships: is a type of GO:0016625 Also known as: 2-ketoglutarate ferredoxin oxidoreductase activity, 2-oxoglutarate ferredoxin oxidoreductase activity, 2-oxoglutarate:ferredoxin 2-oxidoreductase (CoA-succinylating), 2-oxoglutarate:ferredoxin 2-oxidoreductase (decarboxylating), 2-oxoglutarate:ferredoxin oxidoreductase activity, KGOR activity, alpha-ketoglutarate synthase activity, alpha-ketoglutarate-ferredoxin oxidoreductase activity Definition: Catalysis of the reaction: 2-oxoglutarate + CoA + oxidized ferredoxin = succinyl-CoA + CO2 + reduced ferredoxin.